{
  "term_label": "thioredoxin-disulfide reductase (NADPH) activity",
  "gene": "UniProtKB:Q9NNW7",
  "gene_name": "Thioredoxin reductase 2, mitochondrial",
  "term_id": "GO:0004791",
  "gene_symbol": "TXNRD2"
}